microtubule destabilizing activity [GO:0170060] (molecular function) References: PMID:29858272, PMID:36435910 Definition: A protein-containing complex destabilizing activity that promotes microtubule catastrophe (transition from microtubule growth to microtubule shrinkage). Subtypes: microtubule severing ATPase activity [GO:0008568] Relationships: is a type of protein-containing complex destabilizing activity [GO:0140776] Also known as: microtubule catastrophe inducing activity, microtubule catastrophe promoting activity